{
  "gene": "UniProtKB:Q6Y288",
  "gene_symbol": "B3GLCT",
  "gene_name": "Beta-1,3-glucosyltransferase",
  "term_id": "UNKNOWN:0002",
  "term_label": "Unknown biological process"
}